TEAD-YAP complex [GO:0140552] (cellular component) Relationships: is a type of RNA polymerase II transcription regulator complex [GO:0090575] Definition: A transcription factor complex that is composed of the one DNA binding protein of the TEAD family and the transcriptional coactivator YAP. References: PMID:11358867 Sources: GOC:mah Also known as: TEAD-1-YAP complex, TEAD-2 multiprotein complex, TEAD-2-YAP complex, TEAD-3-YAP complex, TEAD-4-YAP complex